{
  "gene_symbol": "MICB",
  "gene_name": "MHC class I polypeptide-related sequence B",
  "term_label": "external side of plasma membrane",
  "gene": "UniProtKB:Q29980",
  "term_id": "GO:0009897"
}